{
  "term_label": "transverse filament",
  "gene_name": "Synaptonemal complex protein 1",
  "gene": "UniProtKB:Q15431",
  "gene_symbol": "SYCP1",
  "term_id": "GO:0000802"
}